regulation of membrane invagination [GO:1905153] (BP) Subtypes: GO:0060099, negative regulation of membrane invagination [GO:1905154], positive regulation of membrane invagination [GO:1905155] Relationships: is a type of GO:0051128; regulates membrane invagination [GO:0010324] Definition: Any process that modulates the frequency, rate or extent of membrane invagination. References: PMID:26589353 Sources: GOC:PARL, GOC:TermGenie, GOC:bf, GO_REF:0000058